negative regulation of cytokine production involved in immune response [GO:0002719] (biological process) Sources: GOC:add Subtypes: negative regulation of B cell cytokine production [GO:0002722], GO:0002725, negative regulation of natural killer cell cytokine production [GO:0002728], negative regulation of dendritic cell cytokine production [GO:0002731], negative regulation of macrophage cytokine production [GO:0010936], negative regulation of mast cell cytokine production [GO:0032764] Also known as: down-regulation of cytokine production during immune response, negative regulation of cytokine biosynthetic process involved in immune response, negative regulation of cytokine secretion involved in immune response, down regulation of cytokine production during immune response, downregulation of cytokine production during immune response, inhibition of cytokine production during immune response, negative regulation of cytokine production during immune response Definition: Any process that stops, prevents, or reduces the frequency, rate, or extent of cytokine production contributing to an immune response. Relationships: is a type of negative regulation of cytokine production [GO:0001818]; is_a negative regulation of production of molecular mediator of immune response [GO:0002701]; is a type of regulation of cytokine production involved in immune response [GO:0002718]; negatively regulates GO:0002367